{
  "gene_symbol": "IL18RAP",
  "term_label": "interleukin-18 receptor activity",
  "gene_name": "Interleukin-18 receptor accessory protein",
  "gene": "UniProtKB:O95256",
  "term_id": "GO:0042008"
}